{
  "gene_symbol": "EDN1",
  "gene_name": "Endothelin-1",
  "term_id": "GO:0014826",
  "term_label": "vein smooth muscle contraction",
  "gene": "UniProtKB:P05305"
}